{
  "gene": "UniProtKB:P0DPE3",
  "term_label": "Unknown cellular component",
  "term_id": "UNKNOWN:0003",
  "gene_name": "Transmembrane and death domain protein 1",
  "gene_symbol": "TMDD1"
}